{
  "term_label": "ventricular cardiac muscle cell action potential",
  "gene_name": "Alpha-1-syntrophin",
  "gene_symbol": "SNTA1",
  "gene": "UniProtKB:Q13424",
  "term_id": "GO:0086005"
}